{
  "gene_symbol": "SRY",
  "term_label": "male sex determination",
  "term_id": "GO:0030238",
  "gene": "UniProtKB:Q05066",
  "gene_name": "Sex-determining region Y protein"
}